{
  "term_label": "extracellular space",
  "gene_symbol": "CXCL13",
  "gene_name": "C-X-C motif chemokine 13",
  "term_id": "GO:0005615",
  "gene": "UniProtKB:O43927"
}